positive regulation of interleukin-25 production [GO:0032749] (biological process) Relationships: is a type of positive regulation of cytokine production [GO:0001819]; is a type of regulation of interleukin-25 production [GO:0032669]; positively regulates GO:0032629 Sources: GOC:mah Definition: Any process that activates or increases the frequency, rate, or extent of interleukin-25 production. Also known as: positive regulation of IL-25 production, up regulation of interleukin-25 production, up-regulation of interleukin-25 production, upregulation of interleukin-25 production, activation of interleukin-25 production, positive regulation of interleukin-25 biosynthetic process, positive regulation of interleukin-25 secretion, stimulation of interleukin-25 production